{
  "gene_name": "B2 bradykinin receptor",
  "gene_symbol": "BDKRB2",
  "term_label": "G protein-coupled receptor signaling pathway",
  "gene": "UniProtKB:P30411",
  "term_id": "GO:0007186"
}